{
  "gene": "UniProtKB:Q00722",
  "term_id": "GO:0005737",
  "gene_symbol": "PLCB2",
  "gene_name": "1-phosphatidylinositol 4,5-bisphosphate phosphodiesterase beta-2",
  "term_label": "cytoplasm"
}